{
  "term_label": "immune receptor activity",
  "gene_name": "Killer cell immunoglobulin-like receptor 2DS4",
  "term_id": "GO:0140375",
  "gene": "UniProtKB:P43632",
  "gene_symbol": "KIR2DS4"
}